{
  "gene_name": "Myocyte-specific enhancer factor 2A",
  "term_id": "UNKNOWN:0003",
  "gene_symbol": "MEF2A",
  "term_label": "Unknown cellular component",
  "gene": "UniProtKB:Q02078"
}